phycobilisome [GO:0030089] (CC) References: PMID:11734882 Sources: GOC:jl, Wikipedia:Phycobilisome Relationships: is a type of GO:0030076; is_a membrane protein complex [GO:0098796]; is part of thylakoid membrane [GO:0042651] Definition: Any of the granules, approximately 32 nm x 48 nm and consisting of highly aggregated phycobiliproteins, that are attached in arrays to the external face of a thylakoid membrane in algae of the phyla Cyanophyta and Rhodophyta, where they function as light-harvesting devices in photosynthesis. Excitation energy in the phycobilisome flows in the sequence: phycoerythrin, phycocyanin, allophycocyanin before passing to the antenna chlorophyll of photosystem II.